{
  "term_label": "positive regulation of phosphatidylinositol 3-kinase/protein kinase B signal transduction",
  "gene": "UniProtKB:Q16288",
  "gene_symbol": "NTRK3",
  "term_id": "GO:0051897",
  "gene_name": "NT-3 growth factor receptor"
}